{
  "term_label": "Unknown cellular component",
  "term_id": "UNKNOWN:0003",
  "gene_name": "Immunoglobulin heavy joining 6 (Fragment)",
  "gene_symbol": "IGHJ6",
  "gene": "UniProtKB:A0A0J9YVP2"
}